{
  "gene_name": "Desert hedgehog protein",
  "gene_symbol": "DHH",
  "term_label": "smoothened signaling pathway",
  "term_id": "GO:0007224",
  "gene": "UniProtKB:O43323"
}